{
  "gene_name": "Endogenous retrovirus group K member 21 Env polyprotein",
  "gene": "UniProtKB:P61565",
  "term_id": "UNKNOWN:0002",
  "gene_symbol": "ERVK-21",
  "term_label": "Unknown biological process"
}